{
  "gene_name": "Mitofusin-1",
  "term_id": "GO:0051646",
  "gene": "UniProtKB:Q8IWA4",
  "gene_symbol": "MFN1",
  "term_label": "mitochondrion localization"
}